{
  "gene_name": "Coiled-coil domain-containing protein 112",
  "term_label": "Unknown molecular function",
  "gene_symbol": "CCDC112",
  "term_id": "UNKNOWN:0001",
  "gene": "UniProtKB:Q8NEF3"
}